{
  "term_id": "GO:0030154",
  "gene_name": "ETS translocation variant 4",
  "gene_symbol": "ETV4",
  "gene": "UniProtKB:P43268",
  "term_label": "cell differentiation"
}